{
  "gene_symbol": "MRPS34",
  "term_id": "GO:0003735",
  "gene_name": "Small ribosomal subunit protein mS34",
  "gene": "UniProtKB:P82930",
  "term_label": "structural constituent of ribosome"
}